{
  "term_id": "UNKNOWN:0001",
  "term_label": "Unknown molecular function",
  "gene_symbol": "GARIN6",
  "gene": "UniProtKB:Q8NEG0",
  "gene_name": "Golgi-associated RAB2 interactor protein 6"
}